{
  "term_id": "GO:0008171",
  "gene": "UniProtKB:Q7Z5W3",
  "gene_name": "RNA 5'-monophosphate methyltransferase",
  "gene_symbol": "BCDIN3D",
  "term_label": "O-methyltransferase activity"
}